Pi Mi complex [GO:0062071] (CC) Definition: A transcription factor complex composed of a homeodomain protein and the M-specific peptide Mi that acts at the regulatory region of genes required for the activation of meiosis. References: PMID:30089908 Relationships: is_a GO:0090575